{
  "gene_name": "Putative heat shock protein HSP 90-beta 2",
  "gene": "UniProtKB:Q58FF8",
  "gene_symbol": "HSP90AB2P",
  "term_label": "cytosol",
  "term_id": "GO:0005829"
}